(E)-beta-ocimene synthase activity [GO:0034768] (molecular function) Relationships: is a type of GO:0016838 Definition: Catalysis of the reaction: geranyl diphosphate = (E)-beta-ocimene + diphosphate. References: PMID:12624761 Sources: EC:4.2.3.106